cell wall polysaccharide catabolic process involved in lateral root development [GO:1902089] (BP) Definition: Any cell wall polysaccharide catabolic process that is involved in lateral root development. References: PMID:23479623 Sources: GOC:TermGenie Also known as: cell wall polysaccharide breakdown involved in lateral root development Relationships: is a type of GO:0044347; is part of lateral root development [GO:0048527]